{
  "gene": "UniProtKB:Q6UXN2",
  "term_id": "GO:0038023",
  "term_label": "signaling receptor activity",
  "gene_name": "Trem-like transcript 4 protein",
  "gene_symbol": "TREML4"
}